{
  "term_label": "Unknown cellular component",
  "term_id": "UNKNOWN:0003",
  "gene": "UniProtKB:Q15928",
  "gene_name": "Zinc finger protein 141",
  "gene_symbol": "ZNF141"
}